{
  "term_id": "GO:0003725",
  "gene_name": "PRKR-interacting protein 1",
  "gene": "UniProtKB:Q9H875",
  "term_label": "double-stranded RNA binding",
  "gene_symbol": "PRKRIP1"
}